{
  "gene_symbol": "GALT",
  "gene_name": "Galactose-1-phosphate uridylyltransferase",
  "term_label": "cytoplasm",
  "term_id": "GO:0005737",
  "gene": "UniProtKB:P07902"
}